{
  "gene_symbol": "CLU",
  "term_label": "extracellular space",
  "term_id": "GO:0005615",
  "gene": "UniProtKB:P10909",
  "gene_name": "Clusterin"
}